{
  "term_id": "GO:0004620",
  "gene_symbol": "DDHD1",
  "gene_name": "Phospholipase DDHD1",
  "gene": "UniProtKB:Q8NEL9",
  "term_label": "phospholipase activity"
}